{
  "gene": "UniProtKB:P42702",
  "gene_name": "Leukemia inhibitory factor receptor",
  "term_id": "GO:0008284",
  "term_label": "positive regulation of cell population proliferation",
  "gene_symbol": "LIFR"
}